{
  "gene_symbol": "OR5L2",
  "gene": "UniProtKB:Q8NGL0",
  "gene_name": "Olfactory receptor 5L2",
  "term_label": "sensory perception of smell",
  "term_id": "GO:0007608"
}